karyogamy involved in conjugation with cellular fusion [GO:0000742] (biological process) Also known as: karyogamy during conjugation with cellular fusion Sources: GOC:elh Relationships: is a type of karyogamy [GO:0000741]; is part of conjugation with cellular fusion [GO:0000747] Definition: During sexual reproduction, the creation of a single nucleus from multiple nuclei as a result of fusing the lipid bilayers that surround each nuclei. This occurs after cytogamy.